cellular response to cold [GO:0070417] (biological process) Sources: GOC:jp Definition: Any process that results in a change in state or activity of a cell (in terms of movement, secretion, enzyme production, gene expression, etc.) as a result of a cold stimulus, a temperature stimulus below the optimal temperature for that organism. Subtypes: cellular response to freezing [GO:0071497] Also known as: cellular response to cold stress Relationships: is a type of GO:0009409; is a type of cellular response to stress [GO:0033554]